{
  "term_label": "bile acid biosynthetic process",
  "gene": "UniProtKB:O75881",
  "gene_symbol": "CYP7B1",
  "gene_name": "Cytochrome P450 7B1",
  "term_id": "GO:0006699"
}